{
  "gene": "UniProtKB:P51148",
  "term_id": "GO:0030139",
  "term_label": "endocytic vesicle",
  "gene_symbol": "RAB5C",
  "gene_name": "Ras-related protein Rab-5C"
}